{
  "term_id": "GO:0032456",
  "gene_name": "EH domain-binding protein 1-like protein 1",
  "term_label": "endocytic recycling",
  "gene_symbol": "EHBP1L1",
  "gene": "UniProtKB:Q8N3D4"
}